{
  "gene": "UniProtKB:Q9NSA2",
  "gene_symbol": "KCND1",
  "term_id": "GO:0045211",
  "gene_name": "Potassium voltage-gated channel subfamily D member 1",
  "term_label": "postsynaptic membrane"
}